{
  "gene_symbol": "RALB",
  "term_label": "plasma membrane",
  "term_id": "GO:0005886",
  "gene_name": "Ras-related protein Ral-B",
  "gene": "UniProtKB:P11234"
}